positive regulation of arbuscule formation for nutrient acquisition from host [GO:0075330] (biological process) Definition: Any process that activates or increases the frequency, rate or extent of symbiont arbuscule formation for nutrient acquisition from host. The host is defined as the larger of the organisms involved in a symbiotic interaction. Sources: GOC:pamgo_curators Note: Note that this term should not be used to annotate gene products of the host. It should only be used to annotate those gene products from the symbiont involved in this process. Relationships: is a type of positive regulation of formation of structure involved in a symbiotic process [GO:0044149]; is a type of GO:0075329; positively regulates formation of arbuscule for nutrient acquisition [GO:0075328]